response to furfural [GO:1901426] (biological process) Definition: Any process that results in a change in state or activity of a cell or an organism (in terms of movement, secretion, enzyme production, gene expression, etc.) as a result of a furfural stimulus. Sources: GOC:TermGenie, GOC:mengo_curators Relationships: is a type of response to oxygen-containing compound [GO:1901700] Regulation: regulated by GO:1901442; negatively regulated by negative regulation of response to furfural [GO:1901443]; RO_0002213 by positive regulation of response to furfural [GO:1901444]